L-alanine biosynthetic process [GO:0042852] (biological process) Definition: The chemical reactions and pathways resulting in the formation of L-alanine, the L-enantiomer of 2-aminopropanoic acid, i.e. (2S)-2-aminopropanoic acid. Sources: GOC:jl, GOC:jsg, GOC:mah Also known as: L-alanine anabolism, L-alanine biosynthesis, L-alanine formation, L-alanine synthesis Relationships: is a type of alanine biosynthetic process [GO:0006523]; is a type of pyruvate family amino acid biosynthetic process [GO:0009079]; is a type of L-alanine metabolic process [GO:0042851] Subtypes: L-alanine biosynthetic process from pyruvate [GO:0019272], L-alanine biosynthetic process via ornithine [GO:0019273]